mono-ADP-D-ribose modification-dependent protein binding [GO:0160003] (molecular function) Note: This term should only be used when the binding is shown to require a mono-ADP-D-ribose post-translational modification: the interaction needs to be tested with and without the PTM. The binding does not need to be at the site of the ADP-D-ribose modification. It may be that the PTM causes a conformational change that allows binding of the protein to another region; this type of modification-dependent protein binding is valid for annotation to this term. Definition: Binding to a protein upon mono-ADP-ribosylation of the target protein. Relationships: is a type of ADP-D-ribose modification-dependent protein binding [GO:0160002] References: PMID:34023495